mating plug formation [GO:0042628] (BP) Relationships: is a type of GO:0022414; is part of insemination [GO:0007320] Definition: The deposition of a plug of sperm or other gelatinous material into the opening of the vulva by a male at the termination of copulation. Probably acts to prevent subsequent matings by other males. Also known as: copulatory plug biosynthesis, copulatory plug deposition, copulatory plug formation, mating plug deposition References: PMID:11267893 Sources: GOC:jl